nucleic acid-protein covalent cross-linking [GO:0018143] (biological process) Sources: GOC:ma Relationships: is a type of GO:0036211 Definition: The formation of a covalent cross-link between a nucleic acid and a protein. Subtypes: GO:0018144